{
  "term_label": "Unknown biological process",
  "gene_name": "Docking protein 6",
  "gene": "UniProtKB:Q6PKX4",
  "gene_symbol": "DOK6",
  "term_id": "UNKNOWN:0002"
}